regulation of metanephric podocyte development [GO:2000477] (biological process) Subtypes: positive regulation of metanephric podocyte development [GO:2000478] Definition: Any process that modulates the frequency, rate or extent of metanephric glomerular visceral epithelial cell development. Relationships: is a type of GO:0060284; regulates metanephric podocyte development [GO:0072249] Sources: GOC:obol Also known as: regulation of metanephric glomerular visceral epithelial cell development